{
  "gene": "UniProtKB:A2VEC9",
  "term_label": "extracellular space",
  "gene_symbol": "SSPOP",
  "term_id": "GO:0005615",
  "gene_name": "SCO-spondin"
}